{
  "gene_name": "Arf-GAP with Rho-GAP domain, ANK repeat and PH domain-containing protein 1",
  "term_label": "trans-Golgi network",
  "gene": "UniProtKB:Q96P48",
  "gene_symbol": "ARAP1",
  "term_id": "GO:0005802"
}